camelliol C synthase activity [GO:0090438] (molecular function) References: PMID:17985917 Sources: GOC:tb Definition: Catalyzes the reaction: (3S)-2,3-epoxy-2,3-dihydrosqualene = camelliol C. Also known as: (3S)-2,3-epoxy-2,3-dihydrosqualene mutase (cyclizing, camelliol-C-forming) Relationships: is a type of intramolecular transferase activity [GO:0016866]